{
  "term_label": "regulation of DNA-templated transcription",
  "gene_name": "Zinc finger protein 679",
  "gene": "UniProtKB:Q8IYX0",
  "term_id": "GO:0006355",
  "gene_symbol": "ZNF679"
}